negative regulation of distal tip cell migration [GO:1903355] (biological process) Relationships: is_a GO:0030336; is a type of regulation of distal tip cell migration [GO:1903354]; negatively regulates distal tip cell migration [GO:0097628] Also known as: down regulation of distal tip cell migration, down-regulation of distal tip cell migration, downregulation of distal tip cell migration, inhibition of distal tip cell migration References: PMID:24968003 Sources: GOC:TermGenie, GOC:mm2, GO_REF:0000058 Definition: Any process that stops, prevents or reduces the frequency, rate or extent of distal tip cell migration.